negative regulation of lymphocyte activation [GO:0051250] (BP) Subtypes: negative regulation of natural killer cell activation [GO:0032815], negative regulation of lymphocyte differentiation [GO:0045620], GO:0050672, negative regulation of T cell activation [GO:0050868], negative regulation of B cell activation [GO:0050869], negative regulation of immunological synapse formation [GO:2000521] Relationships: is a type of GO:0002695; is a type of regulation of lymphocyte activation [GO:0051249]; negatively regulates lymphocyte activation [GO:0046649] Definition: Any process that stops, prevents, or reduces the frequency, rate or extent of lymphocyte activation. Sources: GOC:ai Also known as: down regulation of lymphocyte activation, down-regulation of lymphocyte activation, downregulation of lymphocyte activation, inhibition of lymphocyte activation